regulation of attachment of mitotic spindle microtubules to kinetochore [GO:1902423] (biological process) Definition: Any process that modulates the frequency, rate or extent of attachment of spindle microtubules to kinetochore involved in mitotic sister chromatid segregation. Subtypes: negative regulation of attachment of mitotic spindle microtubules to kinetochore [GO:1902424], positive regulation of attachment of mitotic spindle microtubules to kinetochore [GO:1902425], GO:1905115 Also known as: regulation of attachment of spindle microtubules to kinetochore involved in mitosis, regulation of attachment of spindle microtubules to kinetochore involved in mitotic sister chromatid segregation, regulation of attachment of spindle microtubules to mitotic chromosome, regulation of mitotic attachment of spindle microtubules to kinetochore, regulation of attachment of spindle microtubules to kinetochore during mitosis, regulation of mitotic bipolar attachment References: PMID:22065639 Sources: GOC:TermGenie, GOC:vw Relationships: is a type of GO:0033047; is_a regulation of attachment of spindle microtubules to kinetochore [GO:0051988]; is a type of regulation of metaphase plate congression [GO:0090235]; regulates attachment of mitotic spindle microtubules to kinetochore [GO:0051315]